{
  "gene_symbol": "OR10J4",
  "gene_name": "Olfactory receptor 10J4",
  "gene": "UniProtKB:P0C629",
  "term_label": "odorant binding",
  "term_id": "GO:0005549"
}